 [title]